secretion of lysosomal enzymes [GO:0033299] (biological process) Relationships: is a type of protein secretion [GO:0009306] Definition: The controlled release of lysosomal enzymes by a cell. Sources: GOC:mah Regulation: regulated by regulation of secretion of lysosomal enzymes [GO:0090182]; positively regulated by positive regulation of secretion of lysosomal enzymes [GO:0090340]; negatively regulated by negative regulation of secretion of lysosomal enzymes [GO:0090341] Subtypes: lysosomal enzyme secretion involved in inflammatory response [GO:0002533]